sabinene synthase activity [GO:0080015] (molecular function) References: PMID:12566586, PMID:9747540 Sources: RHEA:68636 Relationships: is a type of cyclase activity [GO:0009975]; is a type of terpene synthase activity [GO:0010333] Definition: Catalysis of the reaction: (2E)-geranyl diphosphate = diphosphate + sabinene.